{
  "gene_name": "Dehydrogenase_reductase SDR family member 2, mitochondrial",
  "gene_symbol": "DHRS2",
  "term_id": "GO:0004090",
  "gene": "UniProtKB:Q13268",
  "term_label": "carbonyl reductase (NADPH) activity"
}